{
  "gene": "UniProtKB:Q8TD57",
  "gene_name": "Dynein axonemal heavy chain 3",
  "term_id": "GO:0008569",
  "gene_symbol": "DNAH3",
  "term_label": "minus-end-directed microtubule motor activity"
}